{
  "gene": "UniProtKB:Q8IY95",
  "gene_name": "Transmembrane protein 192",
  "gene_symbol": "TMEM192",
  "term_label": "lysosomal membrane",
  "term_id": "GO:0005765"
}